2-keto-3-deoxygluconate:proton symporter activity [GO:0015649] (molecular function) Also known as: 2-keto-3-deoxygluconate:hydrogen symporter activity Sources: RHEA:29943, TC:2.A.10.1.1 Relationships: is a type of carbohydrate:proton symporter activity [GO:0005351]; is a type of monosaccharide transmembrane transporter activity [GO:0015145]; is a type of GO:0015355; is part of GO:0046411 Definition: Enables the transfer of a solute or solutes from one side of a membrane to the other according to the reaction: 2-keto-3-deoxygluconate(out) + H+(out) = 2-keto-3-deoxygluconate(in) + H+(in).